negative regulation of cellular response to transforming growth factor beta stimulus [GO:1903845] (biological process) Relationships: is a type of negative regulation of cellular response to growth factor stimulus [GO:0090288]; is_a regulation of cellular response to transforming growth factor beta stimulus [GO:1903844]; negatively regulates cellular response to transforming growth factor beta stimulus [GO:0071560] Definition: Any process that stops, prevents or reduces the frequency, rate or extent of cellular response to transforming growth factor beta stimulus. Also known as: down regulation of cellular response to TGF-beta stimulus, down regulation of cellular response to TGFbeta stimulus, down regulation of cellular response to transforming growth factor beta stimulus, down-regulation of cellular response to TGF-beta stimulus, down-regulation of cellular response to TGFbeta stimulus, down-regulation of cellular response to transforming growth factor beta stimulus, downregulation of cellular response to TGF-beta stimulus, downregulation of cellular response to TGFbeta stimulus, downregulation of cellular response to transforming growth factor beta stimulus, negative regulation of cellular response to TGF-beta stimulus, negative regulation of cellular response to TGFbeta stimulus, inhibition of cellular response to TGF-beta stimulus, inhibition of cellular response to TGFbeta stimulus, inhibition of cellular response to transforming growth factor beta stimulus References: PMID:22269326 Sources: GOC:BHF, GOC:BHF_miRNA, GOC:TermGenie, GOC:rph, GO_REF:0000058